{
  "gene": "UniProtKB:Q9GZW5",
  "term_id": "UNKNOWN:0002",
  "term_label": "Unknown biological process",
  "gene_symbol": "SCAND2P",
  "gene_name": "Putative SCAN domain-containing protein SCAND2P"
}